positive regulation of centriole replication [GO:0046601] (biological process) Relationships: is a type of GO:0046599; is a type of positive regulation of cytoskeleton organization [GO:0051495]; is a type of positive regulation of cell cycle process [GO:0090068]; is a type of positive regulation of organelle assembly [GO:1902117]; positively regulates centriole replication [GO:0007099] Subtypes: positive regulation of centriole elongation [GO:1903724] Sources: GOC:ai Also known as: up regulation of centriole replication, up-regulation of centriole replication, upregulation of centriole replication, activation of centriole replication, stimulation of centriole replication Definition: Any process that activates or increases the frequency, rate or extent of centriole replication.